cellular response to interleukin-11 [GO:0071348] (BP) Sources: GOC:mah Also known as: cellular response to IL-11 Definition: Any process that results in a change in state or activity of a cell (in terms of movement, secretion, enzyme production, gene expression, etc.) as a result of an interleukin-11 stimulus. Relationships: is a type of GO:0071105; is a type of cellular response to cytokine stimulus [GO:0071345]